{
  "term_label": "extracellular space",
  "gene_symbol": "PLOD2",
  "gene": "UniProtKB:O00469",
  "gene_name": "Procollagen-lysine,2-oxoglutarate 5-dioxygenase 2",
  "term_id": "GO:0005615"
}